regulatory T cell apoptotic process [GO:1902482] (BP) Relationships: is a type of GO:0070231 Definition: Any apoptotic process in a regulatory T cell. References: PMID:20471291 Sources: GOC:TermGenie, GOC:nhn Also known as: regulatory T lymphocyte apoptotic process, regulatory T-cell apoptotic process, regulatory T-lymphocyte apoptotic process, regulatory T cell apoptosis, regulatory T lymphocyte apoptosis, regulatory T-cell apoptosis, regulatory T-lymphocyte apoptosis